{
  "gene": "UniProtKB:P0DKX0",
  "term_label": "nucleus",
  "gene_symbol": "ZNF728",
  "gene_name": "Zinc finger protein 728",
  "term_id": "GO:0005634"
}